{
  "term_label": "nucleus",
  "gene": "UniProtKB:Q14586",
  "gene_symbol": "ZNF267",
  "term_id": "GO:0005634",
  "gene_name": "Zinc finger protein 267"
}